carvone reductase activity [GO:0018494] (molecular function) Relationships: is a type of GO:0016627 Sources: EC:1.3.99.25 Definition: Catalysis of the reactions: (1R,4R)-dihydrocarvone + A = (R)-carvone + AH2, and (1R,4S)-isodihydrocarvone + A = (S)-carvone + AH2.